CMP kinase activity [GO:0036430] (molecular function) Relationships: is a type of nucleoside monophosphate kinase activity [GO:0050145] Sources: RHEA:11600 Definition: Catalysis of the reaction: ATP + CMP = ADP + CDP.